regulation of juvenile hormone catabolic process [GO:0045952] (biological process) Sources: GOC:go_curators Relationships: is a type of GO:0019747; is a type of regulation of hormone metabolic process [GO:0032350]; is a type of regulation of lipid catabolic process [GO:0050994]; regulates juvenile hormone catabolic process [GO:0006719] Also known as: regulation of juvenile hormone breakdown, regulation of juvenile hormone catabolism, regulation of juvenile hormone degradation Subtypes: negative regulation of juvenile hormone catabolic process [GO:0045970], positive regulation of juvenile hormone catabolic process [GO:0045971] Definition: Any process that modulates the frequency, rate or extent of the chemical reactions and pathways resulting in the breakdown of juvenile hormone.